{
  "gene_symbol": "DEFB1",
  "term_label": "CCR6 chemokine receptor binding",
  "term_id": "GO:0031731",
  "gene": "UniProtKB:P60022",
  "gene_name": "Beta-defensin 1"
}